{
  "term_id": "GO:0000146",
  "term_label": "microfilament motor activity",
  "gene_symbol": "MYO3B",
  "gene": "UniProtKB:Q8WXR4",
  "gene_name": "Myosin-IIIb"
}